{
  "term_id": "GO:0005737",
  "gene": "UniProtKB:A6NHC0",
  "gene_symbol": "CAPN8",
  "gene_name": "Calpain-8",
  "term_label": "cytoplasm"
}